{
  "term_id": "GO:0000791",
  "term_label": "euchromatin",
  "gene_symbol": "H1-3",
  "gene": "UniProtKB:P16402",
  "gene_name": "Histone H1.3"
}